DNA replication factor C complex [GO:0005663] (cellular component) Definition: A complex that loads the DNA polymerase processivity factor proliferating cell nuclear antigen (PCNA) onto DNA, thereby permitting processive DNA synthesis catalyzed by DNA polymerase. In eukaryotes the complex consists of five polypeptides. Also known as: RFC complex, activator 1 complex Subtypes: cytoplasmic DNA replication factor C complex [GO:0043598], nuclear DNA replication factor C complex [GO:0043599] References: PMID:14614842, PMID:14646196, PMID:16172520 Relationships: is_a protein-containing complex [GO:0032991]; is part of replication fork [GO:0005657]